{
  "term_label": "cytoplasm",
  "term_id": "GO:0005737",
  "gene_name": "Rho guanine nucleotide exchange factor 37",
  "gene_symbol": "ARHGEF37",
  "gene": "UniProtKB:A1IGU5"
}